negative regulation of mitochondrial electron transport, NADH to ubiquinone [GO:1902957] (biological process) Definition: Any process that stops, prevents or reduces the frequency, rate or extent of mitochondrial electron transport, NADH to ubiquinone. Also known as: down regulation of mitochondrial electron transport, NADH to ubiquinone, down regulation of oxidative phosphorylation, NADH to ubiquinone, down-regulation of mitochondrial electron transport, NADH to ubiquinone, down-regulation of oxidative phosphorylation, NADH to ubiquinone, downregulation of mitochondrial electron transport, NADH to ubiquinone, downregulation of oxidative phosphorylation, NADH to ubiquinone, negative regulation of oxidative phosphorylation, NADH to ubiquinone, inhibition of mitochondrial electron transport, NADH to ubiquinone, inhibition of oxidative phosphorylation, NADH to ubiquinone, down regulation of complex I (NADH to ubiquinone), down-regulation of complex I (NADH to ubiquinone), downregulation of complex I (NADH to ubiquinone), inhibition of complex I (NADH to ubiquinone), negative regulation of complex I (NADH to ubiquinone) References: PMID:23530063 Sources: GOC:TermGenie, GOC:dph, GO_REF:0000058 Relationships: is a type of regulation of mitochondrial electron transport, NADH to ubiquinone [GO:1902956]; is a type of negative regulation of mitochondrial ATP synthesis coupled electron transport [GO:1905447]; negatively regulates mitochondrial electron transport, NADH to ubiquinone [GO:0006120]